{
  "gene_symbol": "TNKS2",
  "term_label": "NAD+ poly-ADP-ribosyltransferase activity",
  "gene_name": "Poly [ADP-ribose] polymerase tankyrase-2",
  "term_id": "GO:0003950",
  "gene": "UniProtKB:Q9H2K2"
}